{
  "gene_symbol": "SNRNP200",
  "term_id": "GO:0003723",
  "gene_name": "U5 small nuclear ribonucleoprotein 200 kDa helicase",
  "term_label": "RNA binding",
  "gene": "UniProtKB:O75643"
}